{
  "term_label": "negative regulation of proteolysis",
  "term_id": "GO:0045861",
  "gene": "UniProtKB:P58062",
  "gene_name": "Serine protease inhibitor Kazal-type 7",
  "gene_symbol": "SPINK7"
}